oocyte differentiation [GO:0009994] (BP) Definition: The process in which a relatively unspecialized immature germ cell acquires the specialized features of a mature female gamete. Subtypes: germarium-derived oocyte differentiation [GO:0030706] Relationships: is a type of GO:0003006; is a type of GO:0030154; is part of oogenesis [GO:0048477] Sources: GOC:go_curators, GOC:mtg_sensu Also known as: oocyte cell differentiation